{
  "gene": "UniProtKB:Q86XP0",
  "term_id": "GO:0005509",
  "term_label": "calcium ion binding",
  "gene_name": "Cytosolic phospholipase A2 delta",
  "gene_symbol": "PLA2G4D"
}